{
  "term_id": "GO:0043296",
  "term_label": "apical junction complex",
  "gene_name": "Partitioning defective 3 homolog B",
  "gene_symbol": "PARD3B",
  "gene": "UniProtKB:Q8TEW8"
}